{
  "term_id": "GO:0043542",
  "gene_symbol": "S100P",
  "gene": "UniProtKB:P25815",
  "term_label": "endothelial cell migration",
  "gene_name": "Protein S100-P"
}